Pyrin domain binding [GO:0032090] (molecular function) Sources: GOC:rl Definition: Binding to a Pyrin (PAAD/DAPIN) domain, a protein-protein interaction domain that has the same fold as the Death domain. Relationships: is_a protein domain specific binding [GO:0019904] Also known as: DAPIN domain binding, PAAD domain binding